negative regulation of ornithine catabolic process [GO:1903267] (biological process) Also known as: down regulation of ornithine breakdown, down regulation of ornithine catabolic process, down regulation of ornithine catabolism, down regulation of ornithine degradation, down-regulation of ornithine breakdown, down-regulation of ornithine catabolic process, down-regulation of ornithine catabolism, down-regulation of ornithine degradation, downregulation of ornithine breakdown, downregulation of ornithine catabolic process, downregulation of ornithine catabolism, downregulation of ornithine degradation, negative regulation of ornithine breakdown, negative regulation of ornithine catabolism, negative regulation of ornithine degradation, inhibition of ornithine breakdown, inhibition of ornithine catabolic process, inhibition of ornithine catabolism, inhibition of ornithine degradation References: PMID:12679340 Sources: GOC:TermGenie, GOC:bhm, GO_REF:0000058 Definition: Any process that stops, prevents or reduces the frequency, rate or extent of ornithine catabolic process. Relationships: is a type of negative regulation of catabolic process [GO:0009895]; is_a negative regulation of amino acid metabolic process [GO:0045763]; is a type of GO:0062014; is a type of regulation of ornithine catabolic process [GO:1903266]; negatively regulates L-ornithine catabolic process [GO:0006593] Note: An example of this is ARGI in Saccharomyces cerevisiae (P00812) in PMID:12679340 (inferred from direct assay).